{
  "gene_name": "Histone H2B type F-M",
  "term_label": "structural constituent of chromatin",
  "gene": "UniProtKB:P0C1H6",
  "gene_symbol": "H2BW2",
  "term_id": "GO:0030527"
}